regulation of lipid localization [GO:1905952] (biological process) Subtypes: regulation of lipid transport [GO:0032368], negative regulation of lipid localization [GO:1905953], positive regulation of lipid localization [GO:1905954] Relationships: is a type of regulation of localization [GO:0032879]; regulates lipid localization [GO:0010876] References: PMID:17564681 Sources: GOC:TermGenie, GO_REF:0000058 Also known as: regulation of lipid localisation Definition: Any process that modulates the frequency, rate or extent of lipid localization.